N-acetylcitrulline deacetylase activity [GO:0043909] (molecular function) Relationships: is a type of hydrolase activity, acting on carbon-nitrogen (but not peptide) bonds, in linear amides [GO:0016811] References: PMID:16750290 Sources: GOC:jl, RHEA:61092 Also known as: N-acetyl-L-citrulline deacetylase activity, acetylcitrulline deacetylase activity Definition: Catalysis of the reaction: N-acetyl-L-citrulline + H2O = citrulline + acetate.